{
  "gene": "UniProtKB:Q14236",
  "gene_symbol": "DIAPH2-AS1",
  "term_id": "UNKNOWN:0001",
  "term_label": "Unknown molecular function",
  "gene_name": "Early lymphoid activation gene protein"
}